{
  "gene": "UniProtKB:Q7Z412",
  "gene_symbol": "PEX26",
  "term_id": "GO:0005777",
  "term_label": "peroxisome",
  "gene_name": "Peroxisome assembly protein 26"
}